{
  "gene_symbol": "AK2",
  "term_id": "GO:0004017",
  "gene": "UniProtKB:P54819",
  "term_label": "AMP kinase activity",
  "gene_name": "Adenylate kinase 2, mitochondrial"
}